cytosolic ribosome [GO:0022626] (cellular component) Definition: A ribosome located in the cytosol. Also known as: 70S ribosome, 80S ribosome Relationships: is_a ribosome [GO:0005840]; is part of cytosol [GO:0005829] Sources: GOC:mtg_sensu